{
  "gene_symbol": "SYS1",
  "gene_name": "Protein SYS1 homolog",
  "gene": "UniProtKB:Q8N2H4",
  "term_id": "UNKNOWN:0001",
  "term_label": "Unknown molecular function"
}